{
  "gene": "UniProtKB:P07320",
  "term_label": "visual perception",
  "gene_symbol": "CRYGD",
  "gene_name": "Gamma-crystallin D",
  "term_id": "GO:0007601"
}